acylglycerol transport [GO:0034196] (biological process) Relationships: is a type of lipid transport [GO:0006869] Definition: The directed movement of an acylglycerol into, out of or within a cell, or between cells, by means of some agent such as a transporter or pore. An acylglycerol is any mono-, di- or triester of glycerol with (one or more) fatty acids. Sources: GOC:BHF, GOC:rl Also known as: glyceride transport Regulation: regulated by GO:1901506; negatively regulated by negative regulation of acylglycerol transport [GO:1901507]; positively regulated by positive regulation of acylglycerol transport [GO:1901508] Subtypes: triglyceride transport [GO:0034197]